radial glia-guided pyramidal neuron migration [GO:0140650] (BP) Relationships: is a type of GO:0001764 Subtypes: pyramidal neuron migration to cerebral cortex [GO:0021852] Definition: The radial migration of a pyramidal neuron along radial glial cells. References: PMID:3760547 Also known as: radial glia-dependent neuronal migration